{
  "gene_name": "Phosphatidylglycerophosphatase and protein-tyrosine phosphatase 1",
  "term_id": "GO:0102091",
  "term_label": "phosphatidylinositol-5-phosphate phosphatase activity",
  "gene_symbol": "PTPMT1",
  "gene": "UniProtKB:Q8WUK0"
}